{
  "gene_symbol": "PPP1R32",
  "gene_name": "Protein phosphatase 1 regulatory subunit 32",
  "term_id": "UNKNOWN:0003",
  "term_label": "Unknown cellular component",
  "gene": "UniProtKB:Q7Z5V6"
}